detoxification of zinc ion [GO:0010312] (biological process) Relationships: is a type of detoxification of inorganic compound [GO:0061687]; is part of stress response to zinc ion [GO:1990359] Sources: GOC:tair_curators Definition: Any process that reduces or removes the toxicity of zinc ion. These include transport of zinc away from sensitive areas and to compartments or complexes whose purpose is sequestration of zinc ion.